{
  "gene_symbol": "GCC2",
  "term_id": "GO:0071955",
  "gene_name": "GRIP and coiled-coil domain-containing protein 2",
  "term_label": "recycling endosome to Golgi transport",
  "gene": "UniProtKB:Q8IWJ2"
}